NMDA glutamate receptor clustering [GO:0097114] (biological process) Relationships: is a type of GO:0072578; is part of postsynaptic membrane organization [GO:0001941] References: PMID:15620359 Sources: GOC:BHF, GOC:sjp Also known as: N-methyl-D-aspartate receptor clustering, NMDA receptor clustering Definition: The receptor clustering process in which N-methyl-D-aspartate (NMDA) receptors are localized to distinct domains in the cell membrane.